negative regulation of endodermal cell differentiation [GO:1903225] (biological process) Also known as: down regulation of endoderm cell differentiation, down regulation of endodermal cell differentiation, down-regulation of endoderm cell differentiation, down-regulation of endodermal cell differentiation, downregulation of endoderm cell differentiation, downregulation of endodermal cell differentiation, negative regulation of endoderm cell differentiation, inhibition of endoderm cell differentiation, inhibition of endodermal cell differentiation References: PMID:23154389 Sources: GOC:TermGenie, GOC:als, GO_REF:0000058 Definition: Any process that stops, prevents or reduces the frequency, rate or extent of endodermal cell differentiation. Relationships: is a type of negative regulation of cell differentiation [GO:0045596]; is_a regulation of endodermal cell differentiation [GO:1903224]; negatively regulates endodermal cell differentiation [GO:0035987] Subtypes: negative regulation of endodermal cell fate specification [GO:0042664]